eukaryotic translation initiation factor 2B complex [GO:0005851] (cellular component) References: PMID:9438375 Definition: A multisubunit guanine nucleotide exchange factor which catalyzes the exchange of GDP bound to initiation factor eIF2 for GTP, generating active eIF2-GTP. In humans, it is composed of five subunits, alpha, beta, delta, gamma and epsilon. Also known as: eIF-2B, eif2B Relationships: is a type of guanyl-nucleotide exchange factor complex [GO:0032045]; is part of GO:0005737